{
  "gene_symbol": "CCR8",
  "gene_name": "C-C chemokine receptor type 8",
  "gene": "UniProtKB:P51685",
  "term_id": "GO:0007204",
  "term_label": "positive regulation of cytosolic calcium ion concentration"
}